{
  "gene": "UniProtKB:Q0VAQ4",
  "term_label": "Unknown molecular function",
  "gene_name": "Small cell adhesion glycoprotein",
  "term_id": "UNKNOWN:0001",
  "gene_symbol": "SMAGP"
}